invasive filamentous growth [GO:0036267] (biological process) Also known as: invasive growth References: PMID:22276126 Sources: GOC:di Relationships: is a type of growth of unicellular organism as a thread of attached cells [GO:0070783] Subtypes: invasive growth in response to glucose limitation [GO:0001403], invasive growth in response to heat [GO:0036165], invasive growth in response to pheromone [GO:0045311], GO:0097317, invasive growth in response to abiotic stimulus [GO:0097318] Definition: The growth of colonies in filamentous chains of cells into a substrate.